tubulin complex [GO:0045298] (cellular component) Definition: A heterodimer of tubulins alpha and beta that constitutes the protomer for microtubule assembly. Relationships: is a type of protein-containing complex [GO:0032991]; is part of GO:0005856 Sources: ISBN:0716731363